negative regulation of establishment of protein localization to telomere [GO:1904850] (biological process) Definition: Any process that stops, prevents or reduces the frequency, rate or extent of establishment of protein localization to telomere. References: PMID:25467444 Sources: GOC:BHF, GOC:BHF_telomere, GOC:TermGenie, GOC:nc, GO_REF:0000058 Also known as: down regulation of establishment of protein localisation to telomere, down regulation of establishment of protein localization to chromosome, telomeric region, down regulation of establishment of protein localization to telomere, down-regulation of establishment of protein localisation to telomere, down-regulation of establishment of protein localization to chromosome, telomeric region, down-regulation of establishment of protein localization to telomere, downregulation of establishment of protein localisation to telomere, downregulation of establishment of protein localization to chromosome, telomeric region, downregulation of establishment of protein localization to telomere, negative regulation of establishment of protein localisation to telomere, negative regulation of establishment of protein localization to chromosome, telomeric region, inhibition of establishment of protein localisation to telomere, inhibition of establishment of protein localization to chromosome, telomeric region, inhibition of establishment of protein localization to telomere Relationships: is a type of regulation of establishment of protein localization to telomere [GO:0070203]; is a type of negative regulation of establishment of protein localization [GO:1904950]; negatively regulates GO:0070200